positive regulation of stomatal opening [GO:1902458] (biological process) Definition: Any process that activates or increases the frequency, rate or extent of stomatal opening. Relationships: is a type of positive regulation of cellular process [GO:0048522]; is a type of regulation of stomatal opening [GO:1902456]; positively regulates stomatal opening [GO:1990069] References: PMID:23766366 Sources: GOC:TermGenie Also known as: up regulation of stomatal opening, up-regulation of stomatal opening, upregulation of stomatal opening, activation of stomatal opening